{
  "gene": "UniProtKB:Q99741",
  "term_label": "DNA replication origin binding",
  "gene_symbol": "CDC6",
  "gene_name": "Cell division control protein 6 homolog",
  "term_id": "GO:0003688"
}